{
  "term_id": "UNKNOWN:0003",
  "gene_symbol": "OR9Q2",
  "term_label": "Unknown cellular component",
  "gene": "UniProtKB:Q8NGE9",
  "gene_name": "Olfactory receptor 9Q2"
}